{
  "term_id": "GO:0003975",
  "gene_symbol": "DPAGT1",
  "gene_name": "UDP-N-acetylglucosamine--dolichyl-phosphate N-acetylglucosaminephosphotransferase",
  "gene": "UniProtKB:Q9H3H5",
  "term_label": "UDP-N-acetylglucosamine-dolichyl-phosphate N-acetylglucosaminephosphotransferase activity"
}